negative regulation of G1 to G0 transition [GO:1903451] (biological process) Definition: Any process that stops, prevents or reduces the frequency, rate or extent of G1 to G0 transition. References: PMID:24088570 Sources: GOC:TermGenie, GOC:di, GO_REF:0000058 Also known as: down regulation of G1 to G0 transition, down regulation of G1/G0 transition, down regulation of establishment of cell quiescence, down-regulation of G1 to G0 transition, down-regulation of G1/G0 transition, down-regulation of establishment of cell quiescence, downregulation of G1 to G0 transition, downregulation of G1/G0 transition, downregulation of establishment of cell quiescence, negative regulation of G1/G0 transition, negative regulation of establishment of cell quiescence, inhibition of G1 to G0 transition, inhibition of G1/G0 transition, inhibition of establishment of cell quiescence, down regulation of cell cycle quiescence, down regulation of stationary phase, down-regulation of cell cycle quiescence, down-regulation of stationary phase, downregulation of cell cycle quiescence, downregulation of stationary phase, inhibition of cell cycle quiescence, inhibition of stationary phase, negative regulation of cell cycle quiescence, negative regulation of stationary phase Relationships: is a type of negative regulation of cell cycle process [GO:0010948]; is a type of regulation of G1 to G0 transition [GO:1903450]; negatively regulates GO:0070314